{
  "gene_symbol": "PIGL",
  "term_id": "GO:0005783",
  "gene_name": "N-acetylglucosaminyl-phosphatidylinositol de-N-acetylase",
  "gene": "UniProtKB:Q9Y2B2",
  "term_label": "endoplasmic reticulum"
}